polyenoic fatty acid isomerase activity [GO:0034016] (MF) Relationships: is a type of intramolecular oxidoreductase activity, transposing C=C bonds [GO:0016863] Also known as: (5Z,8Z,11Z,14Z,17Z)-eicosapentaenoate delta8,11-delta7,8-isomerase activity, (5Z,8Z,11Z,14Z,17Z)-eicosapentaenoate delta8,11-delta7,9-isomerase (trans-double-bond-forming) activity, (5Z,8Z,11Z,14Z,17Z)-icosapentaenoate delta8,11-delta7,9-isomerase (trans-double-bond-forming) activity, PFI, eicosapentaenoate cis-delta5,8,11,14,17-eicosapentaenoate cis-delta5-trans-delta7,9-cis-delta14,17 isomerase activity Definition: Catalysis of the reaction: all-cis-icosa-5,8,11,14,17-pentaenoate = (5Z,7E,9E,14Z,17Z)-icosapentaenoate. Sources: RHEA:14889